regulation of actin filament bundle assembly [GO:0032231] (biological process) Also known as: regulation of actin cable assembly, regulation of actin filament bundle formation Definition: Any process that modulates the frequency, rate or extent of the assembly of actin filament bundles. Sources: GOC:mah Relationships: is a type of regulation of cellular component biogenesis [GO:0044087]; is a type of regulation of actin filament organization [GO:0110053]; regulates actin filament bundle assembly [GO:0051017] Subtypes: negative regulation of actin filament bundle assembly [GO:0032232], positive regulation of actin filament bundle assembly [GO:0032233], regulation of stress fiber assembly [GO:0051492], regulation of formin-nucleated actin cable assembly [GO:0090337]